{
  "gene_name": "Paired box protein Pax-1",
  "term_id": "UNKNOWN:0003",
  "gene": "UniProtKB:P15863",
  "term_label": "Unknown cellular component",
  "gene_symbol": "PAX1"
}